symbiont-mediated suppression of host immunoglobulin-mediated immune response [GO:0141140] (biological process) Relationships: is a type of GO:0052562 Definition: A process in which a symbiont interferes with, inhibits or disrupts the normal execution of the immunoglobulin-mediated immune response of the host organism. One common mechanism by which this happens is the direct inhibition of immunoglobulin activity, by direct binding or modification. The host is defined as the larger of the organisms involved in a symbiotic interaction. References: PMID:18426869, PMID:22256861, PMID:24753590 Also known as: symbiont-mediated suppression of host immunoglobulin activity